decanoate-CoA ligase activity [GO:0102391] (molecular function) Sources: GOC:pz, RHEA:33627 Definition: Catalysis of the reaction: ATP + decanoate + CoA = AMP + diphosphate + decanoyl-CoA. Relationships: is a type of medium-chain fatty acid-CoA ligase activity [GO:0031956]